{
  "gene_name": "Pro-glucagon",
  "term_label": "glucagon receptor binding",
  "gene": "UniProtKB:P01275",
  "gene_symbol": "GCG",
  "term_id": "GO:0031769"
}